{
  "gene_symbol": "RTEL1",
  "term_label": "nucleus",
  "gene_name": "Regulator of telomere elongation helicase 1",
  "gene": "UniProtKB:Q9NZ71",
  "term_id": "GO:0005634"
}